{
  "gene": "UniProtKB:Q6ZQY2",
  "term_id": "UNKNOWN:0003",
  "gene_symbol": "LRRC74B",
  "term_label": "Unknown cellular component",
  "gene_name": "Leucine-rich repeat-containing protein 74B"
}